{
  "gene": "UniProtKB:Q04760",
  "term_id": "UNKNOWN:0003",
  "gene_name": "Lactoylglutathione lyase",
  "gene_symbol": "GLO1",
  "term_label": "Unknown cellular component"
}